cyclohydrolase activity [GO:0019238] (molecular function) Sources: GOC:mah Relationships: is a type of hydrolase activity, acting on carbon-nitrogen (but not peptide) bonds, in cyclic amidines [GO:0016814] Subtypes: GTP cyclohydrolase activity [GO:0003933], GO:0003937, methenyltetrahydrofolate cyclohydrolase activity [GO:0004477], GO:0004635, methenyltetrahydromethanopterin cyclohydrolase activity [GO:0018759] Definition: Catalysis of the hydrolysis of any non-peptide carbon-nitrogen bond in a cyclic amidine, a compound of the form R-C(=NH)-NH2, in a reaction that involves the opening of a ring.